{
  "gene_symbol": "CRLF1",
  "term_label": "positive regulation of cell population proliferation",
  "term_id": "GO:0008284",
  "gene_name": "Cytokine receptor-like factor 1",
  "gene": "UniProtKB:O75462"
}